{
  "term_id": "GO:0007229",
  "term_label": "integrin-mediated signaling pathway",
  "gene_name": "Integrin alpha-10",
  "gene": "UniProtKB:O75578",
  "gene_symbol": "ITGA10"
}